{
  "term_label": "N-acetylglucosamine metabolic process",
  "gene_symbol": "CHST2",
  "gene_name": "Carbohydrate sulfotransferase 2",
  "term_id": "GO:0006044",
  "gene": "UniProtKB:Q9Y4C5"
}